{
  "term_id": "GO:0044194",
  "gene_symbol": "GNLY",
  "gene_name": "Granulysin",
  "term_label": "cytolytic granule",
  "gene": "UniProtKB:P22749"
}